{
  "term_id": "GO:0030992",
  "gene_symbol": "CLUAP1",
  "term_label": "intraciliary transport particle B",
  "gene": "UniProtKB:Q96AJ1",
  "gene_name": "Clusterin-associated protein 1"
}